{
  "gene": "UniProtKB:Q5JSH3",
  "gene_symbol": "WDR44",
  "gene_name": "WD repeat-containing protein 44",
  "term_label": "molecular sequestering activity",
  "term_id": "GO:0140313"
}